{
  "term_id": "GO:0000137",
  "gene": "UniProtKB:A6NN73",
  "gene_name": "Golgin subfamily A member 8C",
  "term_label": "Golgi cis cisterna",
  "gene_symbol": "GOLGA8CP"
}